{
  "gene": "UniProtKB:Q96C92",
  "gene_symbol": "ENTR1",
  "term_id": "GO:0036064",
  "term_label": "ciliary basal body",
  "gene_name": "Endosome-associated-trafficking regulator 1"
}